secretory dimeric IgA immunoglobulin complex [GO:0071752] (CC) Note: Note that an IgA immunoglobulin complex has the function of antigen binding if a suitable antigen is available. Dimeric IgA is by far the most common form of polymeric IgA. In human only the IgA1 isotype is capable of a dimeric form. Relationships: is_a dimeric IgA immunoglobulin complex [GO:0071750]; is a type of GO:0071751 Also known as: secretory dimeric IgA antibody, secretory dimeric IgA1 antibody References: PMID:16362985 Sources: GOC:add, ISBN:0781765196 Definition: A dimeric form of secretory IgA immunoglobulin complex.